{
  "gene_name": "Regulation of nuclear pre-mRNA domain-containing protein 1B",
  "term_label": "mRNA 3'-end processing",
  "gene": "UniProtKB:Q9NQG5",
  "term_id": "GO:0031124",
  "gene_symbol": "RPRD1B"
}